inositol hexakisphosphate 5-kinase activity [GO:0000832] (molecular function) Relationships: is a type of GO:0000828 Definition: Catalysis of the reaction: 1D-myo-inositol hexakisphosphate + ATP = 5-diphospho-1D-myo-inositol 1,2,3,4,6-pentakisphosphate + ADP. Also known as: ATP:1D-myo-inositol-hexakisphosphate 5-phosphotransferase activity Sources: RHEA:12793